mesosome [GO:0046868] (cellular component) Relationships: is a type of GO:0110165; is part of plasma membrane [GO:0005886] References: PMID:31921091, PMID:33327493 Definition: An intracellular, often complex, membranous structure, sometimes with additional membranous lamellae inside, found in bacteria. They are associated with synthesis of DNA and secretion of proteins.